convergent extension involved in somitogenesis [GO:0090246] (biological process) Sources: GOC:ascb_2009, GOC:dph, GOC:tb Definition: The morphogenetic process in which a presomitic mesoderm narrows along the left-right axis and lengthens in the rostral-caudal axis contributing to somitogenesis. Relationships: is_a convergent extension involved in gastrulation [GO:0060027]; is a type of convergent extension involved in axis elongation [GO:0060028]; is part of axis elongation involved in somitogenesis [GO:0090245] Regulation: RO_0002211 by GO:1904127; negatively regulated by negative regulation of convergent extension involved in somitogenesis [GO:1904128]; positively regulated by positive regulation of convergent extension involved in somitogenesis [GO:1904129]